ascospore wall beta-glucan biosynthetic process [GO:0034412] (biological process) Definition: The chemical reactions and pathways resulting in the formation of beta-glucans, compounds composed of glucose residues linked by beta-D-glucosidic bonds, found in the walls of ascospores. Subtypes: ascospore wall (1->3)-beta-D-glucan biosynthetic process [GO:0034413] Relationships: is a type of ascospore wall beta-glucan metabolic process [GO:0034408]; is a type of fungal-type cell wall beta-glucan biosynthetic process [GO:0070880] Also known as: ascospore wall beta-glucan anabolism, ascospore wall beta-glucan biosynthesis, ascospore wall beta-glucan formation, ascospore wall beta-glucan synthesis Sources: GOC:mah Regulation: regulated by GO:0060622